regulation of trichoblast fate specification [GO:0010061] (biological process) Sources: GOC:tb Relationships: is_a regulation of cell fate specification [GO:0042659]; is a type of GO:1903888; is a type of regulation of root morphogenesis [GO:2000067]; regulates trichoblast fate specification [GO:0010057] Definition: Any process that modulates trichoblast fate specification. Subtypes: negative regulation of trichoblast fate specification [GO:0010062], positive regulation of trichoblast fate specification [GO:0010063]